{
  "gene_symbol": "SLC7A8",
  "term_label": "neutral L-amino acid transmembrane transporter activity",
  "gene_name": "Large neutral amino acids transporter small subunit 2",
  "gene": "UniProtKB:Q9UHI5",
  "term_id": "GO:0015175"
}